F-actin monooxygenase activity [GO:0120501] (molecular function) Definition: Catalysis of the reaction: L-methionyl-[F-actin] + NADPH + O2 + H+ = L-methionyl-(R)-S-oxide-[F-actin] + NADP+ + H2O. Sources: RHEA:51308 Relationships: is a type of oxidoreductase activity, acting on paired donors, with incorporation or reduction of molecular oxygen, NAD(P)H as one donor, and incorporation of one atom of oxygen [GO:0016709]